Golgi vesicle fusion to target membrane [GO:0048210] (biological process) Also known as: Golgi-derived vesicle fusion to target membrane, dictyosome vesicle fusion to target membrane Subtypes: medial-Golgi-derived vesicle fusion with Golgi trans cisterna membrane [GO:1990672], Golgi medial cisterna-derived vesicle fusion with Golgi cis cisterna membrane [GO:1990690], cis-Golgi-derived vesicle fusion with Golgi medial cisterna membrane [GO:1990691], trans-Golgi-derived vesicle fusion with Golgi medial cisterna membrane [GO:1990692] Definition: The joining of the lipid bilayer membrane around a Golgi transport vesicle to the target lipid bilayer membrane. Relationships: is a type of vesicle fusion [GO:0006906]; is part of GO:0048193 References: PMID:10219233 Sources: GOC:jid, ISBN:0716731363 Regulation: regulated by GO:0048214; positively regulated by positive regulation of Golgi vesicle fusion to target membrane [GO:0048215]; RO_0002212 by negative regulation of Golgi vesicle fusion to target membrane [GO:0048216]